{
  "term_label": "nucleus",
  "gene": "UniProtKB:P41134",
  "term_id": "GO:0005634",
  "gene_name": "DNA-binding protein inhibitor ID-1",
  "gene_symbol": "ID1"
}